{
  "term_label": "external side of plasma membrane",
  "gene_symbol": "ASGR2",
  "term_id": "GO:0009897",
  "gene_name": "Asialoglycoprotein receptor 2",
  "gene": "UniProtKB:P07307"
}